{
  "gene_name": "Keratin, type I cytoskeletal 40",
  "gene": "UniProtKB:Q6A162",
  "term_id": "GO:0005856",
  "gene_symbol": "KRT40",
  "term_label": "cytoskeleton"
}